eisosome membrane domain/MCC [GO:0090512] (CC) Definition: A plasma membrane part that is composed of a furrow-like plasma membrane domain and associated integral transmembrane proteins. References: PMID:22368779 Sources: GOC:al, GOC:vw Relationships: is a type of plasma membrane raft [GO:0044853]; is part of GO:0032126